{
  "term_id": "GO:0000122",
  "gene": "UniProtKB:Q8N895",
  "term_label": "negative regulation of transcription by RNA polymerase II",
  "gene_name": "Zinc finger protein 366",
  "gene_symbol": "ZNF366"
}